{
  "gene_name": "Alpha-ketoglutarate-dependent dioxygenase alkB homolog 4",
  "term_id": "GO:0032451",
  "term_label": "demethylase activity",
  "gene_symbol": "ALKBH4",
  "gene": "UniProtKB:Q9NXW9"
}